{
  "term_id": "UNKNOWN:0002",
  "gene_name": "Uncharacterized protein CXorf65",
  "term_label": "Unknown biological process",
  "gene": "UniProtKB:A6NEN9",
  "gene_symbol": "CXorf65"
}